{
  "gene": "UniProtKB:Q13315",
  "term_id": "GO:0005737",
  "gene_name": "Serine-protein kinase ATM",
  "gene_symbol": "ATM",
  "term_label": "cytoplasm"
}